{
  "term_id": "GO:0005634",
  "gene": "UniProtKB:P47928",
  "gene_symbol": "ID4",
  "term_label": "nucleus",
  "gene_name": "DNA-binding protein inhibitor ID-4"
}